{
  "gene": "UniProtKB:O00160",
  "term_label": "actin cytoskeleton",
  "gene_name": "Unconventional myosin-If",
  "gene_symbol": "MYO1F",
  "term_id": "GO:0015629"
}